{
  "term_label": "chemical synaptic transmission",
  "gene": "UniProtKB:Q13639",
  "term_id": "GO:0007268",
  "gene_symbol": "HTR4",
  "gene_name": "5-hydroxytryptamine receptor 4"
}